regulation of translation [GO:0006417] (biological process) Definition: Any process that modulates the frequency, rate or extent of the chemical reactions and pathways resulting in the formation of proteins by the translation of mRNA or circRNA. Sources: GOC:isa_complete Also known as: regulation of protein anabolism, regulation of protein biosynthesis, regulation of protein formation, regulation of protein synthesis Relationships: is a type of post-transcriptional regulation of gene expression [GO:0010608]; is a type of regulation of protein metabolic process [GO:0051246]; regulates translation [GO:0006412] Subtypes: regulation of translational initiation [GO:0006446], regulation of translational elongation [GO:0006448], regulation of translational termination [GO:0006449], translational readthrough [GO:0006451], translational attenuation [GO:0009386], negative regulation of translation [GO:0017148], GO:0043143, regulation of translation in response to stress [GO:0043555], positive regulation of translation [GO:0045727], regulation of translation, ncRNA-mediated [GO:0045974], regulation of oskar mRNA translation [GO:0046011], regulation of translation involved in anterior/posterior axis specification [GO:0060815], GO:0070129, circadian regulation of translation [GO:0097167], regulation of translation at synapse [GO:0140243], GO:1904803, regulation of cytoplasmic translation [GO:2000765]